{
  "term_id": "GO:0045292",
  "term_label": "mRNA cis splicing, via spliceosome",
  "gene_symbol": "CWC15",
  "gene_name": "Spliceosome-associated protein CWC15 homolog",
  "gene": "UniProtKB:Q9P013"
}